{
  "gene": "UniProtKB:Q15052",
  "gene_name": "Rho guanine nucleotide exchange factor 6",
  "term_id": "GO:0005085",
  "gene_symbol": "ARHGEF6",
  "term_label": "guanyl-nucleotide exchange factor activity"
}